{
  "gene": "UniProtKB:P04035",
  "gene_name": "3-hydroxy-3-methylglutaryl-coenzyme A reductase",
  "gene_symbol": "HMGCR",
  "term_label": "peroxisomal membrane",
  "term_id": "GO:0005778"
}